regulation of microvillus organization [GO:0032530] (biological process) Sources: GOC:mah Also known as: regulation of microvillus organisation, regulation of microvillus organization and biogenesis Relationships: is a type of regulation of plasma membrane bounded cell projection organization [GO:0120035]; regulates microvillus organization [GO:0032528] Subtypes: GO:0032531, GO:0032532, regulation of microvillus assembly [GO:0032534] Definition: Any process that modulates the frequency, rate or extent of a process involved in the formation, arrangement of constituent parts, or disassembly of a microvillus.